{
  "term_label": "CMP-N-acetylneuraminate transmembrane transporter activity",
  "gene_name": "CMP-sialic acid transporter",
  "gene_symbol": "SLC35A1",
  "gene": "UniProtKB:P78382",
  "term_id": "GO:0005456"
}